negative regulation of lamellocyte differentiation [GO:0035204] (biological process) Relationships: is a type of regulation of lamellocyte differentiation [GO:0035203]; is a type of GO:0045611; negatively regulates lamellocyte differentiation [GO:0035171] Also known as: down regulation of lamellocyte differentiation, down-regulation of lamellocyte differentiation, downregulation of lamellocyte differentiation, inhibition of lamellocyte differentiation References: PMID:14734104 Definition: Any process that stops, prevents, or reduces the frequency, rate or extent of lamellocyte differentiation. Lamellocytes differentiate massively in the lymph glands after parasitization and are large flat cells devoted to encapsulation of invaders too large to be phagocytosed by plasmatocytes.